RC-1 DNA recombination complex [GO:0070467] (cellular component) Also known as: DNA recombination complex RC-1, RC-1 complex (recombination complex 1) Relationships: is a type of GO:0140513 References: PMID:8392064, PMID:8670910 Definition: A protein complex that contains DNA ligase III, DNA polymerase epsilon, a 5'-3' exonuclease, and the SMC1 and SMC2 proteins, and is involved in recombinational repair of deletions and gaps in DNA.